{
  "gene": "UniProtKB:Q86VB7",
  "term_id": "GO:0005886",
  "gene_symbol": "CD163",
  "gene_name": "Scavenger receptor cysteine-rich type 1 protein M130",
  "term_label": "plasma membrane"
}